{
  "term_id": "GO:0005525",
  "term_label": "GTP binding",
  "gene": "UniProtKB:P68371",
  "gene_symbol": "TUBB4B",
  "gene_name": "Tubulin beta-4B chain"
}